{
  "gene": "UniProtKB:Q8NC38",
  "gene_name": "Putative uncharacterized protein ZNF436-AS1",
  "term_label": "Unknown biological process",
  "gene_symbol": "ZNF436-AS1",
  "term_id": "UNKNOWN:0002"
}